mitochondrial single-subunit type RNA polymerase binding [GO:0001001] (molecular function) Definition: Binding to a single subunit mitochondrial RNA polymerase enzyme, which is composed of a single catalytic subunit similar to the RNA polymerase enzymes from phages T3, T7, and SP6. Relationships: is a type of GO:0001050 References: PMID:20701995, PMID:2088182 Sources: GOC:txnOH